positive regulation of cholesterol transport [GO:0032376] (biological process) Relationships: is_a positive regulation of sterol transport [GO:0032373]; is a type of regulation of cholesterol transport [GO:0032374]; positively regulates GO:0030301 Definition: Any process that activates or increases the frequency, rate or extent of the directed movement of cholesterol into, out of or within a cell, or between cells, by means of some agent such as a transporter or pore. Sources: GOC:mah Also known as: up regulation of cholesterol transport, up-regulation of cholesterol transport, upregulation of cholesterol transport, activation of cholesterol transport, stimulation of cholesterol transport Subtypes: positive regulation of cholesterol efflux [GO:0010875], GO:0032385, positive regulation of reverse cholesterol transport [GO:1903064], positive regulation of cholesterol import [GO:1904109]